{
  "term_label": "transcription corepressor activity",
  "gene_name": "LIM and cysteine-rich domains protein 1",
  "term_id": "GO:0003714",
  "gene": "UniProtKB:Q9NZU5",
  "gene_symbol": "LMCD1"
}